{
  "gene_symbol": "GGA3",
  "gene_name": "ADP-ribosylation factor-binding protein GGA3",
  "term_id": "GO:0031267",
  "term_label": "small GTPase binding",
  "gene": "UniProtKB:Q9NZ52"
}